regulation of penetration hypha formation [GO:0075202] (BP) Definition: Any process that modulates the frequency, rate or extent of symbiont penetration hypha formation for entry into host. The host is defined as the larger of the organisms involved in a symbiotic interaction. Subtypes: positive regulation of penetration hypha formation [GO:0075203] Relationships: is a type of regulation of anatomical structure morphogenesis [GO:0022603]; is a type of modulation of formation of structure involved in a symbiotic process [GO:0044145]; is a type of modulation by symbiont of entry into host [GO:0052372]; regulates penetration hypha formation [GO:0075201] Also known as: modulation of symbiont penetration hypha formation for entry into host Sources: GOC:pamgo_curators Note: Note that this term should not be used to annotate gene products of the host. It should only be used to annotate those gene products from the symbiont involved in this process.